serotonin secretion by basophil [GO:0002556] (biological process) Definition: The regulated release of serotonin by a basophil or group of basophils. Sources: GOC:add, ISBN:0781735149 Relationships: is a type of GO:0002442; is a type of establishment of localization in cell [GO:0051649]; is a type of GO:0140029; is part of basophil degranulation [GO:0002561] Also known as: serotonin release by basophil